{
  "gene_name": "Syntaxin-19",
  "gene": "UniProtKB:Q8N4C7",
  "term_id": "GO:0000149",
  "term_label": "SNARE binding",
  "gene_symbol": "STX19"
}